{
  "gene": "UniProtKB:Q9H3Q1",
  "gene_name": "Cdc42 effector protein 4",
  "term_label": "Rho protein signal transduction",
  "gene_symbol": "CDC42EP4",
  "term_id": "GO:0007266"
}